{
  "term_label": "positive regulation of apoptotic process",
  "gene": "UniProtKB:Q9HD36",
  "term_id": "GO:0043065",
  "gene_name": "Bcl-2-like protein 10",
  "gene_symbol": "BCL2L10"
}